mitochondrial mRNA catabolic process [GO:0000958] (biological process) Relationships: is a type of GO:0000957; is a type of mRNA catabolic process [GO:0006402] Regulation: regulated by regulation of mitochondrial mRNA catabolic process [GO:1905637]; negatively regulated by GO:1905638; positively regulated by positive regulation of mitochondrial mRNA catabolic process [GO:1905639] Subtypes: mitochondrial mRNA surveillance [GO:0035946] Definition: The chemical reactions and pathways resulting in the breakdown of mRNA transcribed from the mitochondrial genome and occurring in the mitochondrion. Sources: GOC:krc, GOC:mah